{
  "term_label": "Unknown molecular function",
  "term_id": "UNKNOWN:0001",
  "gene_name": "Leucine-rich colipase-like protein 1",
  "gene": "UniProtKB:A6NCL2",
  "gene_symbol": "LRCOL1"
}